activation of immune response [GO:0002253] (BP) Definition: Any process that initiates an immune response. Sources: GOC:add, GO_REF:0000022, ISBN:0781735149 Relationships: is a type of immune system process [GO:0002376]; is a type of positive regulation of immune response [GO:0050778] Subtypes: activation of innate immune response [GO:0002218], immune response-activating signaling pathway [GO:0002757], GO:0006956